{
  "gene_symbol": "RFX3",
  "gene_name": "Transcription factor RFX3",
  "term_label": "DNA-binding transcription factor activity, RNA polymerase II-specific",
  "term_id": "GO:0000981",
  "gene": "UniProtKB:P48380"
}